{
  "gene_symbol": "SERPINC1",
  "term_label": "Unknown biological process",
  "term_id": "UNKNOWN:0002",
  "gene": "UniProtKB:P01008",
  "gene_name": "Antithrombin-III"
}